{
  "term_label": "negative regulation of JNK cascade",
  "term_id": "GO:0046329",
  "gene": "UniProtKB:Q9NYF0",
  "gene_symbol": "DACT1",
  "gene_name": "Dapper homolog 1"
}